regulation of cobalamin metabolic process [GO:0106064] (biological process) Definition: Any process that modulates the frequency, rate or extent of the chemical reactions and pathways involving cobalamin (vitamin B12), a water-soluble vitamin characterized by possession of a corrin nucleus containing a cobalt atom. References: PMID:29056341 Subtypes: positive regulation of cobalamin metabolic process [GO:0106121], negative regulation of cobalamin metabolic process [GO:0106122] Relationships: is a type of regulation of tetrapyrrole metabolic process [GO:1901401]; regulates GO:0009235